{
  "term_id": "UNKNOWN:0002",
  "term_label": "Unknown biological process",
  "gene_name": "Proprotein convertase subtilisin_kexin type 9",
  "gene_symbol": "PCSK9",
  "gene": "UniProtKB:Q8NBP7"
}